epidermal growth factor receptor activity [GO:0005006] (molecular function) Definition: Combining with an epidermal growth factor receptor ligand and transmitting the signal across the plasma membrane to initiate a change in cell activity. Relationships: is a type of transmembrane receptor protein tyrosine kinase activity [GO:0004714]; is part of epidermal growth factor receptor signaling pathway [GO:0007173]; has part epidermal growth factor binding [GO:0048408] Sources: GOC:bf Regulation: negatively regulated by GO:0007175 Also known as: EGF receptor activity, EGFR, TGF-alpha receptor activity, epidermal growth factor-activated receptor activity, transforming growth factor-alpha receptor activity